{
  "term_label": "chromatin binding",
  "term_id": "GO:0003682",
  "gene": "UniProtKB:Q96N64",
  "gene_symbol": "PWWP2A",
  "gene_name": "PWWP domain-containing protein 2A"
}